{
  "term_label": "mitochondrion",
  "term_id": "GO:0005739",
  "gene": "UniProtKB:Q9H2K0",
  "gene_name": "Translation initiation factor IF-3, mitochondrial",
  "gene_symbol": "MTIF3"
}